{
  "term_label": "mitotic cohesin complex",
  "term_id": "GO:0030892",
  "gene": "UniProtKB:Q9UQE7",
  "gene_symbol": "SMC3",
  "gene_name": "Structural maintenance of chromosomes protein 3"
}